regulation of mammary gland epithelial cell proliferation [GO:0033599] (biological process) Definition: Any process that modulates the frequency, rate or extent of mammary gland epithelial cell proliferation. Sources: GOC:mah Relationships: is_a regulation of epithelial cell proliferation [GO:0050678]; RO_0002211 GO:0033598 Subtypes: GO:0033600, GO:0033601, regulation of epithelial cell proliferation involved in mammary gland bud elongation [GO:0060651]